{
  "term_id": "GO:0045944",
  "gene": "UniProtKB:Q92908",
  "gene_symbol": "GATA6",
  "term_label": "positive regulation of transcription by RNA polymerase II",
  "gene_name": "Transcription factor GATA-6"
}